{
  "gene_symbol": "ACSL3",
  "gene": "UniProtKB:O95573",
  "gene_name": "Fatty acid CoA ligase Acsl3",
  "term_id": "GO:0035336",
  "term_label": "long-chain fatty-acyl-CoA metabolic process"
}